autophagosome membrane disassembly [GO:0030399] (biological process) Also known as: autophagic membrane breakdown, autophagic vacuole membrane disassembly, autophagic membrane catabolism, autophagic membrane degradation Relationships: is a type of membrane disassembly [GO:0030397]; is a type of GO:1905037 Sources: GOC:autophagy, GOC:mah Definition: The controlled breakdown of the membranes of autophagosomes.